positive regulation of apoptotic process involved in metanephric nephron tubule development [GO:1900219] (biological process) Relationships: is a type of regulation of apoptotic process involved in metanephric nephron tubule development [GO:1900217]; is a type of positive regulation of apoptotic process involved in development [GO:1904747]; positively regulates apoptotic process involved in metanephric nephron tubule development [GO:1900205] Definition: Any process that activates or increases the frequency, rate or extent of apoptotic process involved in metanephric nephron tubule development. Also known as: activation of apoptotic cell death of metanephric nephron tubule development, activation of apoptotic process of metanephric nephron tubule development, activation of apoptotic programmed cell death of metanephric nephron tubule development, activation of programmed cell death by apoptosis of metanephric nephron tubule development, positive regulation of apoptotic cell death of metanephric nephron tubule development, positive regulation of apoptotic process of metanephric nephron tubule development, positive regulation of apoptotic programmed cell death of metanephric nephron tubule development, positive regulation of programmed cell death by apoptosis of metanephric nephron tubule development, up regulation of apoptotic cell death of metanephric nephron tubule development, up regulation of apoptotic process involved in metanephric nephron tubule development, up regulation of apoptotic process of metanephric nephron tubule development, up regulation of apoptotic programmed cell death of metanephric nephron tubule development, up regulation of programmed cell death by apoptosis of metanephric nephron tubule development, up-regulation of apoptotic cell death of metanephric nephron tubule development, up-regulation of apoptotic process involved in metanephric nephron tubule development, up-regulation of apoptotic process of metanephric nephron tubule development, up-regulation of apoptotic programmed cell death of metanephric nephron tubule development, up-regulation of programmed cell death by apoptosis of metanephric nephron tubule development, upregulation of apoptotic cell death of metanephric nephron tubule development, upregulation of apoptotic process involved in metanephric nephron tubule development, upregulation of apoptotic process of metanephric nephron tubule development, upregulation of apoptotic programmed cell death of metanephric nephron tubule development, upregulation of programmed cell death by apoptosis of metanephric nephron tubule development, activation of apoptosis of metanephric nephron tubule development, activation of apoptotic process involved in metanephric nephron tubule development, activation of apoptotic program of metanephric nephron tubule development, activation of type I programmed cell death of metanephric nephron tubule development, positive regulation of apoptosis of metanephric nephron tubule development, positive regulation of apoptotic program of metanephric nephron tubule development, positive regulation of type I programmed cell death of metanephric nephron tubule development, up regulation of apoptosis of metanephric nephron tubule development, up regulation of apoptotic program of metanephric nephron tubule development, up regulation of type I programmed cell death of metanephric nephron tubule development, up-regulation of apoptosis of metanephric nephron tubule development, up-regulation of apoptotic program of metanephric nephron tubule development, up-regulation of type I programmed cell death of metanephric nephron tubule development, upregulation of apoptosis of metanephric nephron tubule development, upregulation of apoptotic program of metanephric nephron tubule development, upregulation of type I programmed cell death of metanephric nephron tubule development, activation of signaling (initiator) caspase activity of metanephric nephron tubule development, positive regulation of signaling (initiator) caspase activity of metanephric nephron tubule development, up regulation of signaling (initiator) caspase activity of metanephric nephron tubule development, up-regulation of signaling (initiator) caspase activity of metanephric nephron tubule development, upregulation of signaling (initiator) caspase activity of metanephric nephron tubule development References: PMID:17314325 Sources: GOC:TermGenie, GOC:mtg_kidney_jan10, GOC:yaf